{
  "gene_symbol": "CXCL10",
  "term_id": "GO:0006954",
  "gene_name": "C-X-C motif chemokine 10",
  "gene": "UniProtKB:P02778",
  "term_label": "inflammatory response"
}